{
  "gene_name": "Cytoplasmic FMR1-interacting protein 2",
  "gene_symbol": "CYFIP2",
  "gene": "UniProtKB:Q96F07",
  "term_id": "GO:0006915",
  "term_label": "apoptotic process"
}